{
  "term_id": "GO:0045747",
  "gene_symbol": "NEPRO",
  "gene": "UniProtKB:Q6NW34",
  "term_label": "positive regulation of Notch signaling pathway",
  "gene_name": "Nucleolus and neural progenitor protein"
}